{
  "term_id": "UNKNOWN:0001",
  "term_label": "Unknown molecular function",
  "gene": "UniProtKB:Q16864",
  "gene_symbol": "ATP6V1F",
  "gene_name": "V-type proton ATPase subunit F"
}